{
  "gene_name": "Serine_threonine-protein kinase Nek6",
  "term_id": "GO:0007059",
  "gene_symbol": "NEK6",
  "gene": "UniProtKB:Q9HC98",
  "term_label": "chromosome segregation"
}